{
  "gene_name": "T cell receptor beta joining 1-2",
  "gene": "UniProtKB:A0A0J9YX06",
  "term_label": "Unknown biological process",
  "gene_symbol": "TRBJ1-2",
  "term_id": "UNKNOWN:0002"
}